{
  "gene_symbol": "GOLGA8S",
  "term_id": "GO:0032580",
  "gene": "UniProtKB:H3BPF8",
  "term_label": "Golgi cisterna membrane",
  "gene_name": "Golgin subfamily A member 8S"
}